Ddb1-Wdr21 complex [GO:0070913] (cellular component) Definition: A heterodimeric nucleotide-excision repair complex that is involved in transcription-coupled repair. The subunits are known as Ddb1 and Wdr21 in S. pombe; Ddb1 contains a motif called the DDB-box that interacts with adaptor proteins for DDB1/cullin 4 ubiquitin ligases. References: PMID:18794354 Relationships: is a type of nucleotide-excision repair complex [GO:0000109]